{
  "term_id": "GO:0048705",
  "gene_name": "Collagen alpha-1(II) chain",
  "term_label": "skeletal system morphogenesis",
  "gene_symbol": "COL2A1",
  "gene": "UniProtKB:P02458"
}